{
  "gene": "UniProtKB:Q86YS7",
  "term_id": "GO:0005544",
  "term_label": "calcium-dependent phospholipid binding",
  "gene_symbol": "C2CD5",
  "gene_name": "C2 domain-containing protein 5"
}